{
  "gene": "UniProtKB:Q96BD0",
  "term_id": "GO:0015349",
  "gene_name": "Solute carrier organic anion transporter family member 4A1",
  "term_label": "thyroid hormone transmembrane transporter activity",
  "gene_symbol": "SLCO4A1"
}